programmed necrotic cell death [GO:0097300] (biological process) Also known as: regulated necrosis, programmed cell death by necrosis Definition: A necrotic cell death process that results from the activation of endogenous cellular processes, such as signaling involving death domain receptors or Toll-like receptors. References: PMID:21760595 Sources: GOC:mtg_apoptosis Subtypes: necroptotic process [GO:0070266], programmed necrotic cell death in response to starvation [GO:0097385] Note: This term may be used when annotating instances of programmed cell death characterized by necrotic morphology where the involvement of RIPK1 and/or RIPK3 is not shown. See PMID:23818611 for some examples. Relationships: is a type of programmed cell death [GO:0012501] Regulation: regulated by regulation of programmed necrotic cell death [GO:0062098]; negatively regulated by negative regulation of programmed necrotic cell death [GO:0062099]; positively regulated by GO:0062100